{
  "gene_name": "Putative postmeiotic segregation increased 2-like protein 2",
  "term_id": "UNKNOWN:0003",
  "term_label": "Unknown cellular component",
  "gene_symbol": "PMS2P2",
  "gene": "UniProtKB:O95744"
}